negative regulation of ossification [GO:0030279] (biological process) Also known as: down regulation of ossification, down-regulation of ossification, downregulation of ossification, negative regulation of bone biosynthesis, negative regulation of bone formation, inhibition of ossification Relationships: is a type of regulation of ossification [GO:0030278]; is a type of negative regulation of multicellular organismal process [GO:0051241]; negatively regulates GO:0001503 Definition: Any process that stops, prevents, or reduces the frequency, rate or extent of ossification, the formation of bone or of a bony substance or the conversion of fibrous tissue or of cartilage into bone or a bony substance. Sources: GOC:go_curators Subtypes: GO:0030502